{
  "term_label": "olfactory receptor activity",
  "term_id": "GO:0004984",
  "gene": "UniProtKB:Q8NGQ6",
  "gene_symbol": "OR9I1",
  "gene_name": "Olfactory receptor 9I1"
}